regulation of nitric oxide-cGMP mediated signal transduction [GO:0141149] (biological process) Subtypes: positive regulation of nitric oxide-cGMP mediated signal transduction [GO:0141150], negative regulation of nitric oxide-cGMP mediated signal transduction [GO:0141151] Definition: Any process that modulates the rate, frequency or extent of nitric oxide-cGMP mediated signal transduction. References: PMID:35931019 Relationships: is a type of GO:0010749; regulates nitric oxide-cGMP-mediated signaling [GO:0038060]